{
  "gene": "UniProtKB:P78325",
  "term_label": "positive regulation of membrane protein ectodomain proteolysis",
  "gene_name": "Disintegrin and metalloproteinase domain-containing protein 8",
  "gene_symbol": "ADAM8",
  "term_id": "GO:0051044"
}